right lung development [GO:0060458] (biological process) Definition: The biological process whose specific outcome is the progression of a right lung from an initial condition to its mature state. This process begins with the formation of the right lung and ends with the mature structure. The right lung is the lung which is on the right side of the anterior posterior axis looking from a dorsal to ventral aspect. Sources: GOC:dph, GOC:mtg_lung Relationships: is a type of lung development [GO:0030324] Also known as: right pulmonary development